{
  "term_id": "GO:0005886",
  "gene": "UniProtKB:O14763",
  "term_label": "plasma membrane",
  "gene_name": "Tumor necrosis factor receptor superfamily member 10B",
  "gene_symbol": "TNFRSF10B"
}